{
  "gene_name": "KICSTOR complex protein kaptin",
  "term_label": "KICSTOR complex",
  "gene": "UniProtKB:Q9Y664",
  "gene_symbol": "KPTN",
  "term_id": "GO:0140007"
}